prolactin metabolic process [GO:0120122] (biological process) Also known as: prolactin metabolism Relationships: is a type of hormone metabolic process [GO:0042445] Definition: The chemical reactions and pathways involving prolactin, a protein hormone of the anterior pituitary gland that promotes lactation in response to the suckling stimulus of hungry young mammals. References: PMID:11015620